{
  "gene_name": "Caveolin-2",
  "term_id": "GO:0019901",
  "gene_symbol": "CAV2",
  "gene": "UniProtKB:P51636",
  "term_label": "protein kinase binding"
}